{
  "term_id": "GO:0008286",
  "gene_name": "RAC-alpha serine_threonine-protein kinase",
  "gene_symbol": "AKT1",
  "gene": "UniProtKB:P31749",
  "term_label": "insulin receptor signaling pathway"
}